{
  "gene": "UniProtKB:Q9UK39",
  "gene_symbol": "NOCT",
  "term_label": "Unknown biological process",
  "term_id": "UNKNOWN:0002",
  "gene_name": "Nocturnin"
}